{
  "gene": "UniProtKB:P55017",
  "term_id": "GO:0055064",
  "term_label": "chloride ion homeostasis",
  "gene_name": "Solute carrier family 12 member 3",
  "gene_symbol": "SLC12A3"
}